{
  "gene": "UniProtKB:A0A2R8Y619",
  "gene_name": "Histone H2B type 2-K1",
  "gene_symbol": "H2BK1",
  "term_label": "nucleosome",
  "term_id": "GO:0000786"
}